{
  "gene": "UniProtKB:Q53EL6",
  "gene_symbol": "PDCD4",
  "term_label": "Unknown molecular function",
  "gene_name": "Programmed cell death protein 4",
  "term_id": "UNKNOWN:0001"
}